regulation of sequestering of calcium ion [GO:0051282] (biological process) Sources: GOC:ai Definition: Any process that modulates the frequency, rate or extent of the binding or confining calcium ions such that they are separated from other components of a biological system. Also known as: regulation of calcium ion (Ca2+) retention, regulation of calcium ion (Ca2+) sequestering, regulation of calcium ion (Ca2+) sequestration, regulation of calcium ion (Ca2+) storage, regulation of retention of calcium ion (Ca2+), regulation of sequestering of calcium ion (Ca2+), regulation of sequestration of calcium ion (Ca2+), regulation of storage of calcium ion (Ca2+) Subtypes: regulation of release of sequestered calcium ion into cytosol [GO:0051279], GO:0051283, positive regulation of sequestering of calcium ion [GO:0051284] Relationships: is a type of regulation of localization [GO:0032879]; is a type of GO:0050794; regulates GO:0051208